sulfur amino acid metabolic process [GO:0000096] (BP) Relationships: is a type of sulfur compound metabolic process [GO:0006790]; is a type of carboxylic acid metabolic process [GO:0019752] Also known as: sulfur amino acid metabolism, sulphur amino acid metabolic process, sulphur amino acid metabolism Sources: GOC:ai Definition: The chemical reactions and pathways involving amino acids containing sulfur, comprising cysteine, homocysteine, methionine and selenocysteine. Subtypes: sulfur amino acid biosynthetic process [GO:0000097], sulfur amino acid catabolic process [GO:0000098], cysteine metabolic process [GO:0006534], methionine metabolic process [GO:0006555], homocysteine metabolic process [GO:0050667], ergothioneine metabolic process [GO:0052698]